{
  "term_id": "GO:0005615",
  "gene_symbol": "WNT2B",
  "gene_name": "Protein Wnt-2b",
  "term_label": "extracellular space",
  "gene": "UniProtKB:Q93097"
}